{
  "gene": "UniProtKB:Q6UXS9",
  "gene_symbol": "CASP12",
  "term_label": "cytoplasm",
  "term_id": "GO:0005737",
  "gene_name": "Inactive caspase-12"
}